{
  "gene": "UniProtKB:Q9H400",
  "gene_name": "Lck-interacting transmembrane adapter 1",
  "term_label": "protein kinase binding",
  "gene_symbol": "LIME1",
  "term_id": "GO:0019901"
}